{
  "term_label": "microtubule cytoskeleton organization",
  "gene_name": "Tubulin beta 8B",
  "gene": "UniProtKB:A6NNZ2",
  "term_id": "GO:0000226",
  "gene_symbol": "TUBB8B"
}